{
  "gene_name": "Protein argonaute-4",
  "gene_symbol": "AGO4",
  "term_label": "miRNA binding",
  "term_id": "GO:0035198",
  "gene": "UniProtKB:Q9HCK5"
}